{
  "term_id": "GO:0031419",
  "term_label": "cobalamin binding",
  "gene_symbol": "CBLIF",
  "gene": "UniProtKB:P27352",
  "gene_name": "Cobalamin binding intrinsic factor"
}